peptidyl-arginine hydroxylation [GO:0030961] (biological process) Sources: GOC:mah Definition: The hydroxylation of peptidyl-arginine to form peptidyl-hydroxyarginine. Relationships: is_a GO:0018195